{
  "gene": "UniProtKB:A0A1B0GUS4",
  "term_id": "GO:0061631",
  "term_label": "ubiquitin conjugating enzyme activity",
  "gene_name": "Ubiquitin-conjugating enzyme E2 L5",
  "gene_symbol": "UBE2L5"
}